{
  "term_id": "GO:0005634",
  "gene_symbol": "CPHXL",
  "gene": "UniProtKB:A0A1W2PPM1",
  "term_label": "nucleus",
  "gene_name": "Cytoplasmic polyadenylated homeobox-like protein"
}